neomycin biosynthetic process [GO:1901158] (biological process) Sources: GOC:TermGenie, GOC:yaf, MetaCyc:PWY-7016, UniPathway:UPA00969 Relationships: is a type of aminoglycoside antibiotic biosynthetic process [GO:0030648]; is a type of polyol biosynthetic process [GO:0046173] Also known as: neomycin anabolism, neomycin biosynthesis, neomycin formation, neomycin synthesis Definition: The chemical reactions and pathways resulting in the formation of neomycin.